{
  "term_id": "GO:0006644",
  "gene": "UniProtKB:O43688",
  "term_label": "phospholipid metabolic process",
  "gene_symbol": "PLPP2",
  "gene_name": "Phospholipid phosphatase 2"
}